inulosucrase activity [GO:0047725] (MF) Relationships: is a type of hexosyltransferase activity [GO:0016758] Definition: Catalysis of the reaction: sucrose + 2,1-beta-D-fructosyl(n) = glucose + 2,1-beta-D-fructosyl(n+1). Sources: EC:2.4.1.9 Also known as: sucrose 1-fructosyl transferase activity, sucrose 1-fructosyltransferase activity, sucrose:2,1-beta-D-fructan 1-beta-D-fructosyltransferase activity